{
  "gene_name": "Cofilin-2",
  "gene": "UniProtKB:Q9Y281",
  "term_id": "GO:0051014",
  "gene_symbol": "CFL2",
  "term_label": "actin filament severing"
}